{
  "gene_name": "Chromatin target of PRMT1 protein",
  "term_label": "methyl-CpG binding",
  "gene": "UniProtKB:Q9Y3Y2",
  "term_id": "GO:0008327",
  "gene_symbol": "CHTOP"
}